{
  "gene_symbol": "SSU72",
  "gene": "UniProtKB:Q9NP77",
  "term_id": "GO:0008420",
  "term_label": "RNA polymerase II CTD heptapeptide repeat phosphatase activity",
  "gene_name": "RNA polymerase II subunit A C-terminal domain phosphatase SSU72"
}